{
  "gene_name": "Eukaryotic translation initiation factor 3 subunit F",
  "gene": "UniProtKB:O00303",
  "term_id": "GO:0031369",
  "term_label": "translation initiation factor binding",
  "gene_symbol": "EIF3F"
}